{
  "gene_symbol": "MYO18B",
  "gene_name": "Unconventional myosin-XVIIIb",
  "term_label": "Unknown biological process",
  "term_id": "UNKNOWN:0002",
  "gene": "UniProtKB:Q8IUG5"
}